{
  "term_id": "GO:0010507",
  "gene_name": "Ras-related GTP-binding protein B",
  "gene_symbol": "RRAGB",
  "term_label": "negative regulation of autophagy",
  "gene": "UniProtKB:Q5VZM2"
}